{
  "term_id": "GO:0007179",
  "gene": "UniProtKB:P37023",
  "gene_symbol": "ACVRL1",
  "gene_name": "Serine_threonine-protein kinase receptor R3",
  "term_label": "transforming growth factor beta receptor signaling pathway"
}